ethanolamine kinase activity [GO:0004305] (molecular function) Definition: Catalysis of the reaction: ATP + ethanolamine = ADP + 2 H+ + phosphoethanolamine. Sources: EC:2.7.1.82, RHEA:13069 Also known as: ATP:ethanolamine O-phosphotransferase activity, ethanolamine kinase (phosphorylating), ethanolamine phosphokinase activity Relationships: is a type of kinase activity [GO:0016301]; is a type of phosphotransferase activity, alcohol group as acceptor [GO:0016773]